{
  "term_label": "S-formylglutathione hydrolase activity",
  "gene_name": "S-formylglutathione hydrolase",
  "term_id": "GO:0018738",
  "gene": "UniProtKB:P10768",
  "gene_symbol": "ESD"
}